{
  "term_label": "osteoblast differentiation",
  "term_id": "GO:0001649",
  "gene_symbol": "BGLAP",
  "gene": "UniProtKB:P02818",
  "gene_name": "Osteocalcin"
}